{
  "term_id": "UNKNOWN:0002",
  "term_label": "Unknown biological process",
  "gene": "UniProtKB:Q9NW97",
  "gene_symbol": "TMEM51",
  "gene_name": "Transmembrane protein 51"
}